{
  "gene_name": "Paired mesoderm homeobox protein 2B",
  "gene": "UniProtKB:Q99453",
  "term_label": "RNA polymerase II transcription regulatory region sequence-specific DNA binding",
  "gene_symbol": "PHOX2B",
  "term_id": "GO:0000977"
}